{
  "gene_symbol": "SLC11A2",
  "term_id": "GO:0006828",
  "gene_name": "Natural resistance-associated macrophage protein 2",
  "term_label": "manganese ion transport",
  "gene": "UniProtKB:P49281"
}